{
  "gene_name": "RWD domain-containing protein 4",
  "gene_symbol": "RWDD4",
  "term_label": "Unknown molecular function",
  "term_id": "UNKNOWN:0001",
  "gene": "UniProtKB:Q6NW29"
}